{
  "gene_name": "BTB_POZ domain-containing adapter for CUL3-mediated RhoA degradation protein 3",
  "gene": "UniProtKB:Q9H3F6",
  "term_id": "GO:0016567",
  "gene_symbol": "KCTD10",
  "term_label": "protein ubiquitination"
}